{
  "gene_symbol": "BET1L",
  "term_id": "GO:0042147",
  "gene": "UniProtKB:Q9NYM9",
  "term_label": "retrograde transport, endosome to Golgi",
  "gene_name": "BET1-like protein"
}